manganese ion transport [GO:0006828] (biological process) Definition: The directed movement of manganese (Mn) ions into, out of or within a cell, or between cells, by means of some agent such as a transporter or pore. Subtypes: manganese ion transmembrane transport [GO:0071421] Relationships: is a type of transition metal ion transport [GO:0000041] Sources: GOC:ai